{
  "term_label": "extracellular space",
  "gene_name": "Fibrinogen C domain-containing protein 1",
  "term_id": "GO:0005615",
  "gene_symbol": "FIBCD1",
  "gene": "UniProtKB:Q8N539"
}